retrograde trans-synaptic signaling by trans-synaptic protein complex [GO:0098942] (BP) Definition: Cell-cell signaling from postsynapse to presynapse, across the synaptic cleft, mediated by trans-synaptic protein complex. Sources: GOC:dos Relationships: is a type of retrograde trans-synaptic signaling [GO:0098917]; is a type of trans-synaptic signaling by trans-synaptic complex [GO:0099545] Regulation: regulated by regulation of retrograde trans-synaptic signaling by trans-synaptic protein complex [GO:0099176]